{
  "gene": "UniProtKB:Q07817",
  "term_label": "extrinsic apoptotic signaling pathway in absence of ligand",
  "gene_symbol": "BCL2L1",
  "gene_name": "Bcl-2-like protein 1",
  "term_id": "GO:0097192"
}